regulation of protein targeting to membrane [GO:0090313] (biological process) Sources: GOC:tb Definition: Any process that modulates the frequency, rate or extent of the process of directing proteins towards a membrane, usually using signals contained within the protein. Relationships: is a type of regulation of cellular localization [GO:0060341]; is a type of GO:1903533; regulates protein targeting to membrane [GO:0006612] Subtypes: positive regulation of protein targeting to membrane [GO:0090314], GO:0090315, regulation of protein targeting to vacuolar membrane [GO:1900483]